{
  "term_id": "GO:0006357",
  "gene": "UniProtKB:Q96PT3",
  "gene_symbol": "DUX5",
  "term_label": "regulation of transcription by RNA polymerase II",
  "gene_name": "Double homeobox protein 5"
}